{
  "term_label": "oxysterol binding",
  "gene_symbol": "RORC",
  "term_id": "GO:0008142",
  "gene_name": "Nuclear receptor ROR-gamma",
  "gene": "UniProtKB:P51449"
}